{
  "gene": "UniProtKB:P68133",
  "gene_name": "Actin, alpha skeletal muscle",
  "term_id": "GO:0030240",
  "gene_symbol": "ACTA1",
  "term_label": "skeletal muscle thin filament assembly"
}